{
  "term_label": "Unknown biological process",
  "term_id": "UNKNOWN:0002",
  "gene_symbol": "Q8N9L7",
  "gene_name": "Putative uncharacterized protein FLJ36925",
  "gene": "UniProtKB:Q8N9L7"
}